{
  "gene_name": "Telomeric repeat-binding factor 2",
  "gene_symbol": "TERF2",
  "term_label": "protection from non-homologous end joining at telomere",
  "term_id": "GO:0031848",
  "gene": "UniProtKB:Q15554"
}